{
  "term_label": "Unknown molecular function",
  "gene_name": "Chromosome alignment-maintaining phosphoprotein 1",
  "gene_symbol": "CHAMP1",
  "term_id": "UNKNOWN:0001",
  "gene": "UniProtKB:Q96JM3"
}